{
  "gene_symbol": "ST8SIA2",
  "term_id": "GO:0003828",
  "gene": "UniProtKB:Q92186",
  "gene_name": "Alpha-2,8-sialyltransferase 8B",
  "term_label": "alpha-N-acetylneuraminate alpha-2,8-sialyltransferase activity"
}